{
  "gene": "UniProtKB:Q9C0G6",
  "gene_symbol": "DNAH6",
  "term_id": "GO:0051959",
  "gene_name": "Dynein axonemal heavy chain 6",
  "term_label": "dynein light intermediate chain binding"
}